symbiont-mediated induction of tumor or growth in host [GO:0051819] (biological process) Sources: GOC:pg Relationships: is a type of symbiont-mediated perturbation of host cellular process [GO:0044068] Also known as: induction by symbiont of tumor or growth in host, induction by symbiont in host of tumor, nodule, or growth, induction by symbiont in host of tumor, nodule, or growth containing transformed cells, induction by symbiont of nodulation, tumor or growth in host, induction of tumor, nodule, or growth containing transformed cells in other organism during symbiotic interaction, induction of tumor, nodule, or growth containing transformed cells in other organism involved in symbiotic interaction, induction of tumor, nodule, or growth in other organism during symbiotic interaction, induction of tumor, nodule, or growth in other organism involved in symbiotic interaction Definition: The process in which a symbiont causes the formation of a mass of cells in a host organism. While these growths are often called nodules, they are not formed as nitrogen-fixing structures, but rather to provide an environment for the symbiont to grow. In this sense they are parasitic structures rather than mutualistic.